{
  "term_label": "protein maturation",
  "term_id": "GO:0051604",
  "gene_symbol": "KLK9",
  "gene": "UniProtKB:Q9UKQ9",
  "gene_name": "Kallikrein-9"
}